{
  "gene": "UniProtKB:Q8NGG4",
  "gene_symbol": "OR8H1",
  "term_label": "Unknown cellular component",
  "gene_name": "Olfactory receptor 8H1",
  "term_id": "UNKNOWN:0003"
}